{
  "term_id": "GO:0043065",
  "gene_symbol": "DAPK1",
  "term_label": "positive regulation of apoptotic process",
  "gene_name": "Death-associated protein kinase 1",
  "gene": "UniProtKB:P53355"
}